adenylate cyclase-activating G protein-coupled cAMP receptor signaling pathway [GO:0140582] (biological process) Definition: An adenylate cyclase-activating G protein-coupled receptor signaling pathway initiated by extracellular cAMP binding to its receptor on the surface of the target cell, and ending with the regulation of a downstream cellular process. References: PMID:9578623 Also known as: extracellular cAMP signaling pathway Relationships: is a type of adenylate cyclase-activating G protein-coupled receptor signaling pathway [GO:0007189]